maintenance of postsynaptic specialization structure [GO:0098880] (biological process) Sources: GOC:dos Definition: A process which maintains the organization and the arrangement of proteins in the presynaptic specialization. Relationships: is a type of postsynaptic density organization [GO:0097106]; is a type of GO:0099558 Subtypes: maintenance of postsynaptic density structure [GO:0099562]